{
  "term_label": "response to peptide hormone",
  "gene_name": "Signal transducer and activator of transcription 4",
  "gene_symbol": "STAT4",
  "gene": "UniProtKB:Q14765",
  "term_id": "GO:0043434"
}